regulation of ubiquinone biosynthetic process [GO:0010795] (biological process) Definition: Any process that modulates the frequency, rate or extent of ubiquinone biosynthesis. Ubiquinone biosynthesis consists of the chemical reactions and pathways resulting in the formation of ubiquinone, a lipid-soluble electron-transporting coenzyme. Subtypes: negative regulation of ubiquinone biosynthetic process [GO:1904774], positive regulation of ubiquinone biosynthetic process [GO:1904775] Relationships: is a type of regulation of ketone biosynthetic process [GO:0010566]; regulates GO:0006744 Sources: GOC:dph, GOC:tb